{
  "gene_symbol": "UBE2L3",
  "term_label": "protein K11-linked ubiquitination",
  "gene": "UniProtKB:P68036",
  "term_id": "GO:0070979",
  "gene_name": "Ubiquitin-conjugating enzyme E2 L3"
}